{
  "term_id": "GO:1990573",
  "gene": "UniProtKB:Q14500",
  "gene_name": "ATP-sensitive inward rectifier potassium channel 12",
  "gene_symbol": "KCNJ12",
  "term_label": "potassium ion import across plasma membrane"
}